{
  "gene": "UniProtKB:P42081",
  "term_label": "immune response",
  "gene_name": "T-lymphocyte activation antigen CD86",
  "gene_symbol": "CD86",
  "term_id": "GO:0006955"
}